{
  "term_id": "UNKNOWN:0003",
  "gene": "UniProtKB:P38606",
  "gene_name": "V-type proton ATPase catalytic subunit A",
  "term_label": "Unknown cellular component",
  "gene_symbol": "ATP6V1A"
}